{
  "term_label": "clathrin coat assembly",
  "gene_symbol": "NSG2",
  "gene_name": "Neuronal vesicle trafficking-associated protein 2",
  "gene": "UniProtKB:Q9Y328",
  "term_id": "GO:0048268"
}